type 3 galanin receptor binding [GO:0031766] (molecular function) Sources: GOC:mah, GOC:nln Also known as: type 3 galanin receptor ligand Relationships: is a type of GO:0031763 Definition: Binding to a type 3 galanin receptor.